{
  "term_label": "axon guidance",
  "gene_symbol": "MYPN",
  "term_id": "GO:0007411",
  "gene": "UniProtKB:Q86TC9",
  "gene_name": "Myopalladin"
}